{
  "gene_symbol": "AZI2",
  "term_id": "UNKNOWN:0002",
  "gene": "UniProtKB:Q9H6S1",
  "gene_name": "5-azacytidine-induced protein 2",
  "term_label": "Unknown biological process"
}